{
  "term_label": "mitochondrial alanyl-tRNA aminoacylation",
  "gene_symbol": "AARS2",
  "term_id": "GO:0070143",
  "gene_name": "Alanine--tRNA ligase, mitochondrial",
  "gene": "UniProtKB:Q5JTZ9"
}